{
  "gene_name": "Ropporin-1A",
  "term_id": "GO:0031514",
  "gene": "UniProtKB:Q9HAT0",
  "term_label": "motile cilium",
  "gene_symbol": "ROPN1"
}